regulation of chemotaxis [GO:0050920] (biological process) Relationships: is a type of regulation of response to external stimulus [GO:0032101]; is a type of GO:0040012; regulates GO:0006935 Definition: Any process that modulates the frequency, rate or extent of the directed movement of a motile cell or organism in response to a specific chemical concentration gradient. Sources: GOC:ai Subtypes: regulation of leukocyte chemotaxis [GO:0002688], positive regulation of chemotaxis [GO:0050921], negative regulation of chemotaxis [GO:0050922], regulation of negative chemotaxis [GO:0050923], regulation of positive chemotaxis [GO:0050926], GO:0071671, GO:1902667, GO:1904266, regulation of chemotaxis to arachidonate [GO:1904552], regulation of cell chemotaxis to fibroblast growth factor [GO:1904847], regulation of endothelial cell chemotaxis to vascular endothelial growth factor [GO:1904857], regulation of fibroblast chemotaxis [GO:1905210], regulation of astrocyte chemotaxis [GO:2000458], GO:2001026, regulation of muscle cell chemotaxis toward tendon cell [GO:2001281]